Kupffer's vesicle development [GO:0070121] (biological process) Definition: The progression of the Kupffer's vesicle over time from its initial formation until its mature state. The Kupffer's vesicle is a small but distinctive epithelial sac containing fluid, located midventrally posterior to the yolk cell or its extension, and transiently present during most of the segmentation period. Relationships: is a type of anatomical structure development [GO:0048856] Sources: GOC:dgh Also known as: KV development